positive regulation of ERBB signaling pathway [GO:1901186] (biological process) Definition: Any process that activates or increases the frequency, rate or extent of ERBB signaling pathway. Subtypes: positive regulation of epidermal growth factor receptor signaling pathway [GO:0045742], positive regulation of ERBB3 signaling pathway [GO:1905580] Relationships: is a type of positive regulation of signal transduction [GO:0009967]; is a type of regulation of ERBB signaling pathway [GO:1901184]; positively regulates ERBB signaling pathway [GO:0038127] Sources: GOC:BHF, GOC:TermGenie Also known as: activation of EGF receptor family signaling pathway, activation of ERBB signalling pathway, activation of ErbB signaling, positive regulation of EGF receptor family signaling pathway, positive regulation of ERBB signalling pathway, positive regulation of ErbB signaling, up regulation of EGF receptor family signaling pathway, up regulation of ERBB signaling pathway, up regulation of ERBB signalling pathway, up regulation of ErbB signaling, up-regulation of EGF receptor family signaling pathway, up-regulation of ERBB signaling pathway, up-regulation of ERBB signalling pathway, up-regulation of ErbB signaling, upregulation of EGF receptor family signaling pathway, upregulation of ERBB signaling pathway, upregulation of ERBB signalling pathway, upregulation of ErbB signaling, activation of ERBB signaling pathway, activation of EGFR family signaling pathway, positive regulation of EGFR family signaling pathway, up regulation of EGFR family signaling pathway, up-regulation of EGFR family signaling pathway, upregulation of EGFR family signaling pathway